transmembrane-ephrin receptor activity [GO:0005005] (molecular function) Definition: Combining with a transmembrane ephrin to initiate a change in cell activity. References: PMID:9530499 Sources: GOC:mah Relationships: is a type of ephrin receptor activity [GO:0005003] Also known as: transmembrane-Eph receptor activity